positive regulation of chylomicron remodeling [GO:0090319] (biological process) Definition: Any process that increases the rate, frequency, or extent of chylomicron remodeling. Chylomicron remodeling is the acquisition, loss or modification of a protein or lipid within a chylomicron, including the hydrolysis of triglyceride by lipoprotein lipase and the subsequent loss of free fatty acid. Sources: GOC:BHF Also known as: positive regulation of chylomicron remodelling Relationships: is a type of positive regulation of cellular component organization [GO:0051130]; is a type of positive regulation of multicellular organismal process [GO:0051240]; is a type of regulation of chylomicron remodeling [GO:0090318]; positively regulates chylomicron remodeling [GO:0034371]